{
  "gene_symbol": "FOXP4",
  "gene": "UniProtKB:Q8IVH2",
  "gene_name": "Forkhead box protein P4",
  "term_label": "regulation of transcription by RNA polymerase II",
  "term_id": "GO:0006357"
}